{
  "term_id": "GO:0016339",
  "gene": "UniProtKB:Q6ZTQ4",
  "term_label": "calcium-dependent cell-cell adhesion",
  "gene_name": "Cadherin-related family member 3",
  "gene_symbol": "CDHR3"
}